N-acetylglucosamine biosynthetic process [GO:0006045] (biological process) Definition: The chemical reactions and pathways resulting in the formation of N-acetylglucosamine. The D isomer is a common structural unit of glycoproteins in plants, bacteria and animals; it is often the terminal sugar of an oligosaccharide group of a glycoprotein. Also known as: N-acetylglucosamine anabolism, N-acetylglucosamine biosynthesis, N-acetylglucosamine formation, N-acetylglucosamine synthesis Relationships: is a type of GO:0006044; is a type of glucosamine-containing compound biosynthetic process [GO:1901073] Sources: ISBN:0198506732